{
  "gene": "UniProtKB:P18074",
  "term_label": "DNA helicase activity",
  "gene_name": "General transcription and DNA repair factor IIH helicase subunit XPD",
  "gene_symbol": "ERCC2",
  "term_id": "GO:0003678"
}